{
  "gene_name": "Cell division control protein 42 homolog",
  "term_label": "actin filament organization",
  "gene": "UniProtKB:P60953",
  "gene_symbol": "CDC42",
  "term_id": "GO:0007015"
}